regulation of odontogenesis [GO:0042481] (biological process) Relationships: is a type of regulation of animal organ morphogenesis [GO:2000027]; regulates odontogenesis [GO:0042476] Subtypes: positive regulation of odontogenesis [GO:0042482], GO:0042483, regulation of odontogenesis of dentin-containing tooth [GO:0042487] Definition: Any process that modulates the frequency, rate or extent of the formation and development of a tooth or teeth. Sources: GOC:jl Also known as: regulation of tooth development, regulation of odontogenesis of calcareous or chitinous tooth